{
  "gene_symbol": "DPY19L3",
  "term_label": "mannosyltransferase activity",
  "term_id": "GO:0000030",
  "gene": "UniProtKB:Q6ZPD9",
  "gene_name": "Probable C-mannosyltransferase DPY19L3"
}